negative regulation of invasive growth in response to glucose limitation [GO:2000218] (BP) Definition: Any process that stops, prevents, or reduces the frequency, rate or extent of invasive growth in response to glucose limitation. Sources: GOC:mah Relationships: is a type of negative regulation of growth of unicellular organism as a thread of attached cells [GO:0070785]; is a type of GO:2000217; negatively regulates invasive growth in response to glucose limitation [GO:0001403] Also known as: negative regulation of colony morphology